{
  "term_label": "olfactory receptor activity",
  "gene_name": "Olfactory receptor 13C3",
  "gene_symbol": "OR13C3",
  "term_id": "GO:0004984",
  "gene": "UniProtKB:Q8NGS6"
}